{
  "gene_name": "Ribitol-5-phosphate xylosyltransferase 1",
  "gene": "UniProtKB:Q9Y2B1",
  "gene_symbol": "RXYLT1",
  "term_id": "GO:0005794",
  "term_label": "Golgi apparatus"
}